{
  "term_id": "GO:0016226",
  "gene_symbol": "NUBP1",
  "gene": "UniProtKB:P53384",
  "term_label": "iron-sulfur cluster assembly",
  "gene_name": "Cytosolic Fe-S cluster assembly factor NUBP1"
}